{
  "gene_symbol": "HLA-F",
  "gene": "UniProtKB:P30511",
  "term_label": "peptide antigen binding",
  "term_id": "GO:0042605",
  "gene_name": "HLA class I histocompatibility antigen, alpha chain F"
}